{
  "gene_symbol": "PIBF1",
  "gene": "UniProtKB:Q8WXW3",
  "term_label": "microtubule organizing center",
  "gene_name": "Progesterone-induced-blocking factor 1",
  "term_id": "GO:0005815"
}